{
  "gene": "UniProtKB:Q8TEA8",
  "gene_name": "D-aminoacyl-tRNA deacylase 1",
  "term_id": "GO:0005737",
  "gene_symbol": "DTD1",
  "term_label": "cytoplasm"
}